regulation of barbed-end actin filament capping [GO:2000812] (biological process) Relationships: is a type of GO:0030833; is a type of regulation of actin filament depolymerization [GO:0030834]; regulates barbed-end actin filament capping [GO:0051016] Also known as: regulation of barbed-end F-actin capping activity, regulation of barbed-end actin capping activity, regulation of plus-end F-actin capping activity, regulation of plus-end actin filament capping activity Definition: Any process that modulates the frequency, rate or extent of barbed-end actin filament capping. Subtypes: GO:2000813, positive regulation of barbed-end actin filament capping [GO:2000814] Sources: GOC:BHF